negative regulation of root hair elongation [GO:1902891] (biological process) Relationships: is a type of negative regulation of cell growth [GO:0030308]; is a type of negative regulation of developmental growth [GO:0048640]; is_a GO:1902890; is a type of GO:1903430; negatively regulates root hair elongation [GO:0048767] Also known as: down regulation of root hair elongation, down-regulation of root hair elongation, downregulation of root hair elongation, inhibition of root hair elongation Definition: Any process that stops, prevents or reduces the frequency, rate or extent of root hair elongation. References: PMID:22329353 Sources: GOC:TermGenie, GOC:als, GO_REF:0000058